{
  "term_label": "positive regulation of cell population proliferation",
  "gene_symbol": "PRLR",
  "gene_name": "Prolactin receptor",
  "term_id": "GO:0008284",
  "gene": "UniProtKB:P16471"
}